{
  "term_label": "fatty acid elongation",
  "gene_name": "Very-long-chain (3R)-3-hydroxyacyl-CoA dehydratase 2",
  "gene_symbol": "HACD2",
  "term_id": "GO:0030497",
  "gene": "UniProtKB:Q6Y1H2"
}